{
  "term_label": "cytoplasm",
  "gene": "UniProtKB:Q8NFU5",
  "gene_symbol": "IPMK",
  "term_id": "GO:0005737",
  "gene_name": "Inositol polyphosphate multikinase"
}